{
  "term_label": "Unknown molecular function",
  "term_id": "UNKNOWN:0001",
  "gene_name": "Uncharacterized protein",
  "gene": "UniProtKB:A0A2R8Y556",
  "gene_symbol": "A0A2R8Y556"
}